{
  "term_id": "GO:0005765",
  "gene": "UniProtKB:Q86T03",
  "term_label": "lysosomal membrane",
  "gene_name": "Type 1 phosphatidylinositol 4,5-bisphosphate 4-phosphatase",
  "gene_symbol": "PIP4P1"
}